{
  "term_id": "UNKNOWN:0001",
  "gene_name": "Coiled-coil domain-containing protein 63",
  "term_label": "Unknown molecular function",
  "gene_symbol": "CCDC63",
  "gene": "UniProtKB:Q8NA47"
}